GGA codon-amino acid adaptor activity [GO:0033463] (molecular function) Also known as: glycine tRNA Sources: GOC:mah Note: Note that in the standard genetic code, GGA codes for glycine. Definition: A triplet codon-amino acid adaptor activity that recognizes a GGA codon. Relationships: is a type of GO:0030533